{
  "gene_name": "Cadherin-20",
  "gene": "UniProtKB:Q9HBT6",
  "term_id": "GO:0016339",
  "term_label": "calcium-dependent cell-cell adhesion",
  "gene_symbol": "CDH20"
}